{
  "gene_symbol": "LIMD2",
  "term_id": "GO:0051015",
  "gene": "UniProtKB:Q9BT23",
  "term_label": "actin filament binding",
  "gene_name": "LIM domain-containing protein 2"
}